{
  "term_label": "RNA polymerase II cis-regulatory region sequence-specific DNA binding",
  "gene": "UniProtKB:A0A0U1RQI7",
  "gene_name": "Kruppel-like factor 18",
  "term_id": "GO:0000978",
  "gene_symbol": "KLF18"
}